positive regulation of mast cell activation [GO:0033005] (biological process) Subtypes: positive regulation of mast cell activation involved in immune response [GO:0033008], GO:0038097 Sources: GOC:mah Definition: Any process that activates or increases the frequency, rate, or extent of mast cell activation. Relationships: is a type of positive regulation of leukocyte activation [GO:0002696]; is a type of regulation of mast cell activation [GO:0033003]; RO_0002213 mast cell activation [GO:0045576]